{
  "term_id": "GO:0051011",
  "gene": "UniProtKB:Q14980",
  "gene_symbol": "NUMA1",
  "gene_name": "Nuclear mitotic apparatus protein 1",
  "term_label": "microtubule minus-end binding"
}